putrescine biosynthetic process from arginine [GO:0033388] (biological process) Sources: GOC:mah Subtypes: putrescine biosynthetic process from arginine, via ornithine [GO:0033387], GO:0033389, GO:0033390 Definition: The chemical reactions and pathways resulting in the formation of putrescine, 1,4-diaminobutane, from other compounds, including arginine. Relationships: is a type of arginine metabolic process [GO:0006525]; is a type of glutamine family amino acid metabolic process [GO:0009064]; is a type of putrescine biosynthetic process [GO:0009446] Also known as: putrescine anabolism from arginine, putrescine biosynthesis from arginine, putrescine formation from arginine, putrescine synthesis from arginine